cGMP catabolic process [GO:0046069] (biological process) Definition: The chemical reactions and pathways resulting in the breakdown of cyclic GMP, guanosine 3',5'-phosphate. Sources: GOC:go_curators Also known as: cGMP breakdown, cGMP catabolism, cGMP degradation Relationships: is_a purine ribonucleotide catabolic process [GO:0009154]; is_a GO:0009214; is a type of cGMP metabolic process [GO:0046068]